URM1 ligase activity [GO:0061667] (molecular function) Relationships: is a type of URM1 transferase activity [GO:0042294]; is a type of ubiquitin-like protein ligase activity [GO:0061659] Definition: Catalysis of the transfer of URM1 to a substrate protein via the reaction X-URM1 + S = X + S-URM1, where X is either an E2 or E3 enzyme, the X-URM1 linkage is a thioester bond, and the S-URM1 linkage is an isopeptide bond between the C-terminal amino acid of URM1 and the epsilon-amino group of lysine residues in the substrate. Also known as: E3 Sources: GOC:dph